{
  "term_id": "UNKNOWN:0002",
  "gene": "UniProtKB:O43427",
  "term_label": "Unknown biological process",
  "gene_symbol": "FIBP",
  "gene_name": "Acidic fibroblast growth factor intracellular-binding protein"
}